high-density lipoprotein particle clearance [GO:0034384] (biological process) Definition: The process in which a high-density lipoprotein particle is removed from the blood via receptor-mediated endocytosis and its constituent parts degraded. Regulation: regulated by GO:0010982; positively regulated by positive regulation of high-density lipoprotein particle clearance [GO:0010983]; negatively regulated by negative regulation of high-density lipoprotein particle clearance [GO:0010987] Also known as: HDL clearance Sources: GOC:BHF, GOC:mah Relationships: is a type of plasma lipoprotein particle clearance [GO:0034381]